{
  "gene": "UniProtKB:P23511",
  "gene_name": "Nuclear transcription factor Y subunit alpha",
  "gene_symbol": "NFYA",
  "term_label": "DNA-binding transcription factor activity, RNA polymerase II-specific",
  "term_id": "GO:0000981"
}